{
  "term_label": "poly-ADP-D-ribose binding",
  "gene_symbol": "RNF146",
  "gene": "UniProtKB:Q9NTX7",
  "gene_name": "E3 ubiquitin-protein ligase RNF146",
  "term_id": "GO:0072572"
}